{
  "gene_name": "C-C motif chemokine 19",
  "gene": "UniProtKB:Q99731",
  "term_label": "chemokine-mediated signaling pathway",
  "term_id": "GO:0070098",
  "gene_symbol": "CCL19"
}